equatorial microtubule organization [GO:0031121] (biological process) Also known as: equatorial microtubule organisation, equatorial microtubule organization and biogenesis Sources: GOC:mah, GOC:vw Definition: A process that is carried out at the cellular level which results in the assembly, arrangement of constituent parts, or disassembly of structures formed of microtubules and associated proteins at the midpoint of a cell. Subtypes: GO:0031025 Relationships: is a type of microtubule cytoskeleton organization [GO:0000226]